collagen binding involved in cell-matrix adhesion [GO:0098639] (molecular function) Sources: GOC:dos Relationships: is_a collagen binding [GO:0005518]; is a type of GO:0098634 Definition: Any collagen binding that occurs as part of cell-matrix adhesion.